aerobic respiration, using carbon monoxide as electron donor [GO:0019410] (BP) Definition: The metabolic process in which carbon monoxide (CO) is oxidized to carbon dioxide (CO2) to generate energy. Conservation of energy in this process likely uses sodium ion gradients for ATP synthesis and is coupled to quantitative sulfide methylation. Relationships: is a type of aerobic respiration [GO:0009060]; is a type of GO:0015975 References: PMID:18024677